{
  "term_label": "Unknown biological process",
  "gene_name": "Protein YIPF2",
  "gene": "UniProtKB:Q9BWQ6",
  "term_id": "UNKNOWN:0002",
  "gene_symbol": "YIPF2"
}